nuclear progesterone receptor binding [GO:0033142] (molecular function) Definition: Binding to a nuclear progesterone receptor. Relationships: is a type of nuclear receptor binding [GO:0016922] Also known as: progesterone receptor binding Sources: GOC:mah